stretch-activated, monoatomic cation-selective, calcium channel activity [GO:0015275] (molecular function) Definition: Enables the transmembrane transfer of a calcium ion by a channel that opens in response to a mechanical stress in the form of stretching. Relationships: is a type of calcium channel activity [GO:0005262]; is a type of mechanosensitive monoatomic cation channel activity [GO:0140135] Subtypes: stretch-activated, monoatomic cation-selective, calcium channel activity involved in regulation of action potential [GO:0097364] Sources: GOC:mtg_transport Also known as: stretch-activated, cation-selective, calcium channel activity